{
  "gene": "UniProtKB:P62070",
  "term_label": "GTPase activity",
  "gene_name": "Ras-related protein R-Ras2",
  "term_id": "GO:0003924",
  "gene_symbol": "RRAS2"
}